{
  "gene": "UniProtKB:P58743",
  "gene_name": "Prestin",
  "term_id": "GO:1902476",
  "gene_symbol": "SLC26A5",
  "term_label": "chloride transmembrane transport"
}